cellular_component [GO:0005575] (cellular component) Sources: GOC:pdt Definition: A location, relative to cellular compartments and structures, occupied by a macromolecular machine. There are three types of cellular components described in the gene ontology: (1) the cellular anatomical entity where a gene product carries out a molecular function (e.g., plasma membrane, cytoskeleton) or membrane-enclosed compartments (e.g., mitochondrion); (2) virion components, where viral proteins act, and (3) the stable macromolecular complexes of which gene product are parts (e.g., the clathrin complex). Also known as: cell or subcellular entity, cellular component, subcellular entity Subtypes: protein-containing complex [GO:0032991], virion component [GO:0044423], cellular anatomical structure [GO:0110165] Note: Note that, in addition to forming the root of the cellular component ontology, this term is recommended for the annotation of gene products whose cellular component is unknown. When this term is used for annotation, it indicates that no information was available about the cellular component of the gene product annotated as of the date the annotation was made; the evidence code 'no data' (ND), is used to indicate this.